mitochondrial inner membrane fusion [GO:1990627] (biological process) Also known as: mitochondrion inner membrane fusion References: PMID:17055438 Sources: GOC:vw Relationships: is a type of GO:0007007; BFO_0000050 mitochondrial fusion [GO:0008053] Definition: The membrane organization process that joins two mitochondrial inner membranes to form a single membrane.